{
  "term_label": "chromosome segregation",
  "gene_symbol": "DLGAP5",
  "gene": "UniProtKB:Q15398",
  "term_id": "GO:0007059",
  "gene_name": "Disks large-associated protein 5"
}